L-amino acid transport [GO:0015807] (biological process) Subtypes: L-alanine transport [GO:0015808], L-cystine transport [GO:0015811], L-leucine transport [GO:0015820], GO:0015824, GO:0015825, tyrosine transport [GO:0015828], L-glutamate import [GO:0051938], histamine secretion, neurotransmission [GO:0061538], L-lysine transport [GO:1902022], GO:1902024, L-alpha-amino acid transmembrane transport [GO:1902475] Sources: GOC:ai, GOC:jsg, GOC:mah Definition: The directed movement of L-enantiomer amino acids into, out of or within a cell, or between cells, by means of some agent such as a transporter or pore. Relationships: is a type of GO:0006865; is a type of carboxylic acid transport [GO:0046942]; is a type of nitrogen compound transport [GO:0071705]